{
  "gene": "UniProtKB:Q9UKN1",
  "term_id": "UNKNOWN:0001",
  "term_label": "Unknown molecular function",
  "gene_symbol": "MUC12",
  "gene_name": "Mucin-12"
}